{
  "term_id": "GO:0045202",
  "gene_symbol": "ACTG1",
  "gene_name": "Actin, cytoplasmic 2",
  "term_label": "synapse",
  "gene": "UniProtKB:P63261"
}